negative regulation of myelination [GO:0031642] (biological process) Also known as: down regulation of myelination, down-regulation of myelination, downregulation of myelination, inhibition of myelination Sources: GOC:mah Definition: Any process that stops, prevents, or reduces the frequency, rate or extent of the formation of a myelin sheath around nerve axons. Relationships: is a type of regulation of myelination [GO:0031641]; is a type of negative regulation of nervous system process [GO:0031645]; is a type of negative regulation of cellular process [GO:0048523]; negatively regulates GO:0042552